venom-mediated perturbation of G protein-coupled receptor signaling pathway [GO:0044513] (biological process) Also known as: envenomation resulting in modulation of G protein-coupled receptor activity in other organism, envenomation resulting in modulation of G-protein coupled receptor activity in other organism, envenomation resulting in modulation of G protein-coupled receptor activity in another organism Definition: A process in which an organism alters or subverts a G protein-coupled receptor signaling pathway in another organism via the action of a venom. Relationships: is a type of venom-mediated perturbation of signal transduction [GO:0044509] Subtypes: venom-mediated activation of G protein-coupled receptor signaling pathway [GO:0044514], GO:0140162, venom-mediated suppression of bradykinin-dependent vasodilation [GO:0140163] References: PMID:8405712 Sources: GOC:fj, GOC:jl